negative regulation of interleukin-27-mediated signaling pathway [GO:0070108] (biological process) Relationships: is_a negative regulation of cytokine-mediated signaling pathway [GO:0001960]; is a type of regulation of interleukin-27-mediated signaling pathway [GO:0070107]; negatively regulates GO:0070106 Also known as: negative regulation of IL-27-mediated signaling pathway, negative regulation of IL27RA/IL6ST signaling pathway, negative regulation of interleukin-27-mediated signalling pathway Sources: GOC:BHF, GOC:mah Definition: Any process that decreases the rate, frequency or extent of an interleukin-27-mediated signaling pathway.